{
  "term_id": "GO:0005634",
  "gene": "UniProtKB:Q15004",
  "term_label": "nucleus",
  "gene_name": "PCNA-associated factor",
  "gene_symbol": "PCLAF"
}